negative regulation of spinal cord association neuron differentiation [GO:1902830] (biological process) Relationships: is a type of GO:0045665; is a type of regulation of spinal cord association neuron differentiation [GO:1902829]; negatively regulates spinal cord association neuron differentiation [GO:0021527] References: PMID:21730158 Sources: GOC:TermGenie, GOC:mr, GO_REF:0000058 Also known as: down regulation of spinal cord association neuron differentiation, down regulation of spinal cord dorsal interneuron differentiation, down-regulation of spinal cord association neuron differentiation, down-regulation of spinal cord dorsal interneuron differentiation, downregulation of spinal cord association neuron differentiation, downregulation of spinal cord dorsal interneuron differentiation, negative regulation of spinal cord dorsal interneuron differentiation, inhibition of spinal cord association neuron differentiation, inhibition of spinal cord dorsal interneuron differentiation Definition: Any process that stops, prevents or reduces the frequency, rate or extent of spinal cord association neuron differentiation.